regulation of mitotic spindle pole body separation [GO:0010695] (biological process) Definition: Any process that modulates the rate, frequency or extent of the process involving the release of duplicated mitotic spindle pole bodies (SPBs) and their migration away from each other within the nuclear membrane. Also known as: regulation of SPB separation References: PMID:16792804, PMID:18500339 Sources: GOC:dph, GOC:tb Subtypes: positive regulation of mitotic spindle pole body separation [GO:0010696], negative regulation of mitotic spindle pole body separation [GO:0010697] Relationships: is a type of regulation of cell cycle process [GO:0010564]; regulates GO:0000073